{
  "term_id": "GO:0005886",
  "gene": "UniProtKB:Q8NG77",
  "term_label": "plasma membrane",
  "gene_name": "Olfactory receptor 2T12",
  "gene_symbol": "OR2T12"
}